{
  "gene_symbol": "PFN4",
  "term_id": "UNKNOWN:0002",
  "term_label": "Unknown biological process",
  "gene_name": "Profilin-4",
  "gene": "UniProtKB:Q8NHR9"
}